ascorbate glutathione cycle [GO:0033355] (biological process) Relationships: is a type of glutathione metabolic process [GO:0006749]; is a type of L-ascorbic acid metabolic process [GO:0019852]; is a type of GO:0042744 Sources: GOC:mah, MetaCyc:PWY-2261 Also known as: hydrogen peroxide detoxification Definition: A cyclic series of interconversions involving L-ascorbate and glutathione that scavenges hydrogen peroxide and reduces it to water, with concomitant oxidation of NADPH.